{
  "term_id": "GO:0030018",
  "gene": "UniProtKB:Q9NP98",
  "term_label": "Z disc",
  "gene_name": "Myozenin-1",
  "gene_symbol": "MYOZ1"
}